{
  "gene_symbol": "ANXA2P2",
  "gene": "UniProtKB:A6NMY6",
  "gene_name": "Putative annexin A2-like protein",
  "term_label": "nucleus",
  "term_id": "GO:0005634"
}